{
  "gene": "UniProtKB:Q86Y78",
  "gene_name": "Ly6_PLAUR domain-containing protein 6",
  "term_id": "GO:0090263",
  "gene_symbol": "LYPD6",
  "term_label": "positive regulation of canonical Wnt signaling pathway"
}